{
  "gene_symbol": "ZZZ3",
  "term_id": "UNKNOWN:0003",
  "term_label": "Unknown cellular component",
  "gene": "UniProtKB:Q8IYH5",
  "gene_name": "ZZ-type zinc finger-containing protein 3"
}